sinoatrial node cell fate commitment [GO:0060930] (biological process) Also known as: SA node cell commitment, SAN cell commitment, sinus node cell commitment Sources: GOC:mtg_heart Relationships: is a type of cardiac pacemaker cell fate commitment [GO:0060927]; BFO_0000050 sinoatrial node cell differentiation [GO:0060921] Definition: The commitment of cells to sinoatrial (SA) node cell fates and their capacity to differentiate into SA node cells. SA node cells are pacemaker cells that are found in the sinoatrial node.